secretion by lung epithelial cell involved in lung growth [GO:0061033] (biological process) Also known as: fetal lung liquid secretion Definition: The controlled release of liquid by a lung epithelial cell that contributes to an increase in size of the lung as part of its development. Relationships: is a type of secretion by cell [GO:0032940]; is part of lung growth [GO:0060437] Sources: GOC:dph